{
  "term_id": "GO:0045944",
  "gene_name": "Transcription factor SOX-7",
  "gene": "UniProtKB:Q9BT81",
  "term_label": "positive regulation of transcription by RNA polymerase II",
  "gene_symbol": "SOX7"
}